negative regulation of interleukin-10 production [GO:0032693] (biological process) Sources: GOC:mah Relationships: is a type of GO:0001818; is a type of GO:0032653; negatively regulates interleukin-10 production [GO:0032613] Definition: Any process that stops, prevents, or reduces the frequency, rate, or extent of interleukin-10 production. Also known as: down regulation of interleukin-10 production, down-regulation of interleukin-10 production, downregulation of interleukin-10 production, negative regulation of IL-10 production, inhibition of interleukin-10 production, negative regulation of interleukin-10 biosynthetic process, negative regulation of interleukin-10 secretion